{
  "term_label": "Unknown molecular function",
  "gene": "UniProtKB:Q9BQA1",
  "term_id": "UNKNOWN:0001",
  "gene_name": "Methylosome protein WDR77",
  "gene_symbol": "WDR77"
}